benzaldehyde dehydrogenase (NADP+) activity [GO:0018477] (molecular function) Also known as: NADP-linked benzaldehyde dehydrogenase, benzaldehyde:NADP+ oxidoreductase Definition: Catalysis of the reaction: benzaldehyde + NADP+ + H2O = benzoate + NADPH + H+. Relationships: is a type of aldehyde dehydrogenase (NADP+) activity [GO:0033721] Sources: RHEA:21660